{
  "term_label": "axon",
  "term_id": "GO:0030424",
  "gene_symbol": "POTEKP",
  "gene": "UniProtKB:Q9BYX7",
  "gene_name": "Putative beta-actin-like protein 3"
}